{
  "term_id": "GO:0005925",
  "term_label": "focal adhesion",
  "gene_symbol": "LIMS2",
  "gene_name": "LIM and senescent cell antigen-like-containing domain protein 2",
  "gene": "UniProtKB:Q7Z4I7"
}